MCM complex loading [GO:0140530] (biological process) Relationships: is_a cell cycle process [GO:0022402]; is a type of protein-DNA complex assembly [GO:0065004]; is part of nuclear cell cycle DNA replication initiation [GO:1902315] References: PMID:23603117, PMID:28191893, PMID:28191894, PMID:28501329 Also known as: MCM complex loading at replication origin, MCM double hexamer formation at replication origin Definition: The protein localization process in which two MCM complexes become associated with chromatin at replication origins. MCM loading begins when origin-bound ORC and Cdc6 (Cdc18 in fission yeast) recruit one MCM2-7/Cdt1 complex to the origin, includes formation of a succession of intermediate complexes and ATP hydrolysis-dependent Mcm2-7 ring closure, and ends when two MCM hexamers fully encircle DNA, and are oriented head-to-head. The double hexamer is inactive for DNA unwinding. MCM loading takes place during G1 phase, and precedes CMG complex assembly.